{
  "gene": "UniProtKB:A5A3E0",
  "term_id": "GO:0016020",
  "gene_name": "POTE ankyrin domain family member F",
  "gene_symbol": "POTEF",
  "term_label": "membrane"
}